{
  "term_label": "Unknown biological process",
  "term_id": "UNKNOWN:0002",
  "gene_name": "Tetratricopeptide repeat protein 22",
  "gene_symbol": "TTC22",
  "gene": "UniProtKB:Q5TAA0"
}